{
  "gene_name": "Interferon regulatory factor 7",
  "gene_symbol": "IRF7",
  "term_label": "nucleus",
  "term_id": "GO:0005634",
  "gene": "UniProtKB:Q92985"
}